{
  "gene": "UniProtKB:Q96AQ2",
  "term_label": "Unknown cellular component",
  "gene_name": "Transmembrane protein 125",
  "gene_symbol": "TMEM125",
  "term_id": "UNKNOWN:0003"
}